{
  "term_id": "GO:0061512",
  "gene": "UniProtKB:O00294",
  "gene_name": "Tubby-related protein 1",
  "gene_symbol": "TULP1",
  "term_label": "protein localization to cilium"
}